monoterpenoid metabolic process [GO:0016098] (biological process) Subtypes: GO:0016099, GO:0016100 Also known as: monoterpenoid metabolism Relationships: is_a terpenoid metabolic process [GO:0006721] Sources: ISBN:0198547684 Definition: The chemical reactions and pathways involving monoterpenoid compounds, terpenoids having a C10 skeleton.